{
  "term_id": "GO:0005737",
  "gene": "UniProtKB:P42338",
  "gene_name": "Phosphatidylinositol 4,5-bisphosphate 3-kinase catalytic subunit beta isoform",
  "term_label": "cytoplasm",
  "gene_symbol": "PIK3CB"
}